{
  "gene_symbol": "DOK4",
  "term_label": "cell surface receptor protein tyrosine kinase signaling pathway",
  "gene": "UniProtKB:Q8TEW6",
  "term_id": "GO:0007169",
  "gene_name": "Docking protein 4"
}